{
  "gene_name": "CD40 ligand",
  "term_label": "cytokine activity",
  "gene_symbol": "CD40LG",
  "gene": "UniProtKB:P29965",
  "term_id": "GO:0005125"
}